{
  "gene_name": "Forkhead box protein D2",
  "gene_symbol": "FOXD2",
  "term_id": "GO:0000978",
  "term_label": "RNA polymerase II cis-regulatory region sequence-specific DNA binding",
  "gene": "UniProtKB:O60548"
}